{
  "gene": "UniProtKB:Q96A26",
  "gene_name": "Protein FAM162A",
  "term_label": "Unknown molecular function",
  "gene_symbol": "FAM162A",
  "term_id": "UNKNOWN:0001"
}